dextrin dextranase activity [GO:0050103] (molecular function) Also known as: 1,4-alpha-D-glucan:1,6-alpha-D-glucan 6-alpha-D-glucosyltransferase activity, dextran dextrinase activity, dextrin 6-glucosyltransferase activity Relationships: is a type of hexosyltransferase activity [GO:0016758] Sources: EC:2.4.1.2, MetaCyc:DEXTRIN-DEXTRANASE-RXN Definition: Catalysis of the reaction: 1,4-alpha-D-glucosyl(n) + 1,6-alpha-D-glucosyl(m) = 1,4-alpha-D-glucosyl(n-1) + 1,6-alpha-D-glucosyl(m+1).